{
  "term_id": "GO:0003714",
  "term_label": "transcription corepressor activity",
  "gene": "UniProtKB:Q92802",
  "gene_name": "NEDD4-binding protein 2-like 2",
  "gene_symbol": "N4BP2L2"
}